{
  "gene_symbol": "PAK1IP1",
  "term_id": "GO:0005730",
  "gene": "UniProtKB:Q9NWT1",
  "term_label": "nucleolus",
  "gene_name": "p21-activated protein kinase-interacting protein 1"
}